{
  "gene_symbol": "CXorf51B",
  "term_label": "Unknown molecular function",
  "term_id": "UNKNOWN:0001",
  "gene_name": "Uncharacterized protein CXorf51B",
  "gene": "UniProtKB:P0DPH9"
}